nitrogen catabolite regulation of transcription from RNA polymerase II promoter [GO:0001079] (biological process) Definition: A transcription regulation process in which the presence of one nitrogen source leads to the modulation of the frequency, rate, or extent of transcription, from an RNA polymerase II promoter, of specific genes involved in the metabolism of other nitrogen sources. Relationships: is a type of GO:0006357; is a type of nitrogen catabolite regulation of transcription [GO:0090293] References: PMID:19104072 Sources: GOC:mah, GOC:txnOH Also known as: regulation of transcription from RNA polymerase II promoter by nitrogen catabolites Subtypes: nitrogen catabolite activation of transcription from RNA polymerase II promoter [GO:0001080], nitrogen catabolite repression of transcription from RNA polymerase II promoter [GO:0001081]